nitrate reductase (cytochrome) activity [GO:0050140] (molecular function) Relationships: is_a GO:0008940; is a type of oxidoreductase activity, acting on a heme group of donors, nitrogenous group as acceptor [GO:0016677] Definition: Catalysis of the reaction: 2 Fe(II)-[cytochrome] + nitrate + 2 H+ = 2 Fe(III)-[cytochrome] + nitrite + H2O. Sources: RHEA:12909 Also known as: benzyl viologen-nitrate reductase activity, ferrocytochrome:nitrate oxidoreductase activity